{
  "gene": "UniProtKB:Q13434",
  "term_label": "ubiquitin protein ligase activity",
  "term_id": "GO:0061630",
  "gene_name": "Putative E3 ubiquitin-protein ligase makorin-4",
  "gene_symbol": "MKRN4P"
}